L-glutamine catabolic process [GO:0006543] (BP) Sources: GOC:ai Also known as: glutamine breakdown, glutamine catabolism, glutamine degradation Relationships: is a type of GO:0006541; is a type of GO:0170035; is_a proteinogenic amino acid catabolic process [GO:0170040] Definition: The chemical reactions and pathways resulting in the breakdown of L-glutamine, 2-amino-4-carbamoylbutanoic acid.